{
  "gene": "UniProtKB:P47928",
  "term_id": "GO:0000122",
  "term_label": "negative regulation of transcription by RNA polymerase II",
  "gene_name": "DNA-binding protein inhibitor ID-4",
  "gene_symbol": "ID4"
}